{
  "gene": "UniProtKB:Q29983",
  "term_label": "external side of plasma membrane",
  "gene_name": "MHC class I polypeptide-related sequence A",
  "gene_symbol": "MICA",
  "term_id": "GO:0009897"
}